{
  "term_id": "GO:0022857",
  "gene_name": "Solute carrier family 15 member 5",
  "gene_symbol": "SLC15A5",
  "gene": "UniProtKB:A6NIM6",
  "term_label": "transmembrane transporter activity"
}